{
  "term_label": "cytosolic large ribosomal subunit",
  "gene_symbol": "RPL3L",
  "gene_name": "Ribosomal protein uL3-like",
  "term_id": "GO:0022625",
  "gene": "UniProtKB:Q92901"
}